{
  "gene_name": "Cytosolic carboxypeptidase 3",
  "term_id": "GO:0015631",
  "term_label": "tubulin binding",
  "gene": "UniProtKB:Q8NEM8",
  "gene_symbol": "AGBL3"
}